{
  "gene_symbol": "BTBD18",
  "term_label": "transposable element silencing",
  "term_id": "GO:0010526",
  "gene_name": "BTB_POZ domain-containing protein 18",
  "gene": "UniProtKB:B2RXH4"
}